{
  "gene": "UniProtKB:Q6RI45",
  "gene_symbol": "BRWD3",
  "gene_name": "Bromodomain and WD repeat-containing protein 3",
  "term_label": "regulation of transcription by RNA polymerase II",
  "term_id": "GO:0006357"
}